{
  "term_id": "UNKNOWN:0001",
  "term_label": "Unknown molecular function",
  "gene_symbol": "TTC9C",
  "gene": "UniProtKB:Q8N5M4",
  "gene_name": "Tetratricopeptide repeat protein 9C"
}